transition metal ion binding [GO:0046914] (molecular function) Subtypes: GO:0005506, GO:0005507, GO:0008270, nickel cation binding [GO:0016151], manganese ion binding [GO:0030145], molybdenum ion binding [GO:0030151], GO:0045340, GO:0046870, cobalt ion binding [GO:0050897], vanadium ion binding [GO:0051212] Definition: Binding to a transition metal ions; a transition metal is an element whose atom has an incomplete d-subshell of extranuclear electrons, or which gives rise to a cation or cations with an incomplete d-subshell. Transition metals often have more than one valency state. Biologically relevant transition metals include vanadium, manganese, iron, copper, cobalt, nickel, molybdenum and silver. Sources: ISBN:0198506732 Relationships: is a type of metal ion binding [GO:0046872]